{
  "term_label": "Unknown cellular component",
  "gene_symbol": "FKBPL",
  "term_id": "UNKNOWN:0003",
  "gene_name": "FK506-binding protein-like",
  "gene": "UniProtKB:Q9UIM3"
}